serine-type endopeptidase complex [GO:1905370] (cellular component) Definition: A protein complex which is capable of serine-type endopeptidase activity. Note: An example of this is PLAU in human (UniProt symbol P00749) in PMID:1689240 (inferred from direct assay). Subtypes: GO:0005787, mitochondrial inner membrane peptidase complex [GO:0042720] Relationships: is a type of serine-type peptidase complex [GO:1905286]; is a type of GO:1905369 References: PMID:1689240 Sources: GOC:TermGenie, GOC:bhm, GO_REF:0000088